{
  "gene_symbol": "HOXA9",
  "gene_name": "Homeobox protein Hox-A9",
  "gene": "UniProtKB:P31269",
  "term_id": "GO:0009952",
  "term_label": "anterior/posterior pattern specification"
}